{
  "term_id": "GO:0005615",
  "gene": "UniProtKB:P13671",
  "gene_symbol": "C6",
  "term_label": "extracellular space",
  "gene_name": "Complement component C6"
}